{
  "gene_symbol": "COQ2",
  "gene_name": "4-hydroxybenzoate polyprenyltransferase, mitochondrial",
  "gene": "UniProtKB:Q96H96",
  "term_label": "mitochondrial inner membrane",
  "term_id": "GO:0005743"
}